fructose import across plasma membrane [GO:1990539] (biological process) Also known as: fructose uptake, fructose import Definition: The directed movement of fructose substance from outside of a cell, across the plasma membrane and into the cytosol. Relationships: is a type of fructose transmembrane transport [GO:0015755]; is a type of GO:0140271 References: PMID:10735857